cellular response to palmitoleic acid [GO:1904927] (biological process) References: PMID:25429233 Sources: GOC:TermGenie, GOC:mr, GO_REF:0000071 Definition: Any process that results in a change in state or activity of a cell (in terms of movement, secretion, enzyme production, gene expression, etc.) as a result of a palmitoleic acid stimulus. Relationships: is a type of cellular response to fatty acid [GO:0071398]; is a type of response to palmitoleic acid [GO:1904926]